aminotriazole:proton antiporter activity [GO:0015314] (molecular function) Definition: Enables the transfer of a solute or solutes from one side of a membrane to the other according to the reaction: H+(out) + aminotriazole(in) = H+(in) + aminotriazole(out). Sources: TC:2.A.1.3.1 Also known as: aminotriazole:hydrogen antiporter activity Relationships: is a type of GO:0045119; is_a aminotriazole transmembrane transporter activity [GO:1901478]